{
  "gene_symbol": "SEPHS2",
  "term_id": "GO:0005737",
  "gene_name": "Selenide, water dikinase 2",
  "gene": "UniProtKB:Q99611",
  "term_label": "cytoplasm"
}